metanephric proximal tubule morphogenesis [GO:0072288] (biological process) Definition: The process in which the anatomical structures of a metanephric proximal tubule are generated and organized. The metanephric proximal tubule is a metanephric nephron tubule that connects Bowman's capsule to the descending thin limb of the loop of Henle in the metanephros. It has a brush border epithelial morphology. Relationships: is a type of proximal tubule morphogenesis [GO:0072158]; is a type of metanephric nephron tubule morphogenesis [GO:0072282]; is part of metanephric proximal tubule development [GO:0072237] Sources: GOC:mtg_kidney_jan10